{
  "term_id": "GO:0005178",
  "term_label": "integrin binding",
  "gene_name": "Endothelial cell-specific molecule 1",
  "gene": "UniProtKB:Q9NQ30",
  "gene_symbol": "ESM1"
}